alpha6-beta4 integrin-Fyn complex [GO:0071098] (cellular component) Definition: A protein complex that consists of an alpha6-beta4 integrin complex bound to the Src family tyrosine kinase Fyn. References: PMID:11684709 Also known as: ITGA6-ITGB4-FYN complex Relationships: is_a GO:0098797